Sertoli cell apoptotic process [GO:1902484] (biological process) Relationships: is_a epithelial cell apoptotic process [GO:1904019] References: PMID:17761895 Sources: GOC:TermGenie, GOC:ic Also known as: Sertoli cell apoptosis Definition: Any apoptotic process in a Sertoli cell.